{
  "gene_symbol": "TECTB",
  "term_label": "extracellular matrix structural constituent",
  "gene_name": "Beta-tectorin",
  "term_id": "GO:0005201",
  "gene": "UniProtKB:Q96PL2"
}